{
  "term_label": "Unknown cellular component",
  "term_id": "UNKNOWN:0003",
  "gene": "UniProtKB:Q9UHP6",
  "gene_symbol": "RSPH14",
  "gene_name": "Radial spoke head 14 homolog"
}